{
  "term_label": "nuclear-transcribed mRNA catabolic process",
  "gene_symbol": "EXOSC2",
  "term_id": "GO:0000956",
  "gene": "UniProtKB:Q13868",
  "gene_name": "Exosome complex component RRP4"
}